{
  "gene_symbol": "FMOD",
  "term_label": "Unknown biological process",
  "gene": "UniProtKB:Q06828",
  "gene_name": "Fibromodulin",
  "term_id": "UNKNOWN:0002"
}